{
  "term_label": "propionyl-CoA carboxylase activity",
  "term_id": "GO:0004658",
  "gene_symbol": "PCCA",
  "gene_name": "Propionyl-CoA carboxylase alpha chain, mitochondrial",
  "gene": "UniProtKB:P05165"
}